{
  "gene_name": "Single-stranded DNA-binding protein 4",
  "term_label": "transcription coactivator activity",
  "gene": "UniProtKB:Q9BWG4",
  "gene_symbol": "SSBP4",
  "term_id": "GO:0003713"
}